inositol hexakisphosphate 6-kinase activity [GO:0000831] (molecular function) Relationships: is a type of inositol hexakisphosphate kinase activity [GO:0000828] Definition: Catalysis of the reaction: ATP + 1D-myo-inositol hexakisphosphate = ADP + 6-diphospho-1D-myo-inositol (1,2,3,4,5)pentakisphosphate. References: PMID:16429326 Sources: GOC:elh